{
  "gene_name": "Mitochondrial proton_calcium exchanger protein",
  "term_id": "GO:0006851",
  "gene_symbol": "LETM1",
  "gene": "UniProtKB:O95202",
  "term_label": "mitochondrial calcium ion transmembrane transport"
}